{
  "term_id": "GO:0023019",
  "gene": "UniProtKB:Q8N907",
  "term_label": "signal transduction involved in regulation of gene expression",
  "gene_name": "DAN domain family member 5",
  "gene_symbol": "DAND5"
}